negative regulation of MAP kinase activity [GO:0043407] (biological process) Relationships: is a type of regulation of MAP kinase activity [GO:0043405]; is a type of negative regulation of MAPK cascade [GO:0043409]; is a type of negative regulation of protein serine/threonine kinase activity [GO:0071901]; RO_0002212 MAP kinase activity [GO:0004707] Definition: Any process that stops, prevents, or reduces the frequency, rate or extent of MAP kinase activity. Subtypes: negative regulation of JUN kinase activity [GO:0043508] Sources: GOC:dph, GOC:go_curators Also known as: down regulation of MAPK activity, down-regulation of MAPK activity, downregulation of MAPK activity, negative regulation of mitogen activated protein kinase activity, negative regulation of mitogen-activated protein kinase activity, inhibition of MAPK activity